germ cell nucleus [GO:0043073] (cellular component) Definition: The nucleus of a germ cell, a reproductive cell in multicellular organisms. Relationships: is a type of nucleus [GO:0005634] Subtypes: male germ cell nucleus [GO:0001673], female germ cell nucleus [GO:0001674] Sources: CL:0000586, GOC:go_curators Also known as: germ-cell nucleus